{
  "gene_name": "Small nuclear ribonucleoprotein Sm D2",
  "gene": "UniProtKB:P62316",
  "term_id": "GO:0046540",
  "gene_symbol": "SNRPD2",
  "term_label": "U4/U6 x U5 tri-snRNP complex"
}